{
  "gene": "UniProtKB:O43423",
  "gene_name": "Putative uncharacterized protein ANP32CP",
  "term_id": "GO:0048471",
  "gene_symbol": "ANP32CP",
  "term_label": "perinuclear region of cytoplasm"
}